{
  "gene_name": "Phosphoinositide 3-kinase regulatory subunit 4",
  "term_id": "GO:0034272",
  "gene": "UniProtKB:Q99570",
  "gene_symbol": "PIK3R4",
  "term_label": "phosphatidylinositol 3-kinase complex, class III, type II"
}